{
  "term_id": "GO:0003689",
  "gene": "UniProtKB:Q8WVB6",
  "gene_symbol": "CHTF18",
  "term_label": "DNA clamp loader activity",
  "gene_name": "Chromosome transmission fidelity protein 18 homolog"
}